{
  "gene_name": "UDP-GlcNAc:betaGal beta-1,3-N-acetylglucosaminyltransferase 9",
  "gene_symbol": "B3GNT9",
  "gene": "UniProtKB:Q6UX72",
  "term_id": "GO:0000139",
  "term_label": "Golgi membrane"
}